{
  "gene_name": "BTB_POZ domain-containing protein KCTD3",
  "gene": "UniProtKB:Q9Y597",
  "term_label": "Unknown cellular component",
  "term_id": "UNKNOWN:0003",
  "gene_symbol": "KCTD3"
}